{
  "term_label": "RNA polymerase II cis-regulatory region sequence-specific DNA binding",
  "term_id": "GO:0000978",
  "gene_name": "CCAAT_enhancer-binding protein epsilon",
  "gene": "UniProtKB:Q15744",
  "gene_symbol": "CEBPE"
}